{
  "term_label": "Unknown molecular function",
  "gene_name": "Follistatin-related protein 4",
  "gene": "UniProtKB:Q6MZW2",
  "term_id": "UNKNOWN:0001",
  "gene_symbol": "FSTL4"
}